plasmodesmatal plasma membrane [GO:0009548] (cellular component) Relationships: is a type of cellular anatomical structure [GO:0110165]; is part of plasma membrane [GO:0005886]; is part of plasmodesma [GO:0009506] Sources: GOC:mah Definition: The portion of the plasma membrane surrounding a plasmodesma.